{
  "term_id": "GO:0016435",
  "gene_symbol": "BUD23",
  "term_label": "rRNA (guanine) methyltransferase activity",
  "gene": "UniProtKB:O43709",
  "gene_name": "Probable 18S rRNA (guanine-N(7))-methyltransferase"
}